{
  "gene": "UniProtKB:Q9BZF9",
  "term_label": "Unknown molecular function",
  "gene_name": "Uveal autoantigen with coiled-coil domains and ankyrin repeats",
  "gene_symbol": "UACA",
  "term_id": "UNKNOWN:0001"
}